endothelium development [GO:0003158] (biological process) Relationships: is a type of epithelium development [GO:0060429] Sources: GOC:mtg_heart Subtypes: GO:0061147, GO:0072011 Definition: The process whose specific outcome is the progression of an endothelium over time, from its formation to the mature structure. Endothelium refers to the layer of cells lining blood vessels, lymphatics, the heart, and serous cavities, and is derived from bone marrow or mesoderm. Corneal endothelium is a special case, derived from neural crest cells.